vestibular receptor cell differentiation [GO:0060114] (biological process) Also known as: vestibular hair cell differentiation Sources: GOC:dph Relationships: is a type of GO:0035315; is a type of inner ear receptor cell differentiation [GO:0060113] Definition: The process in which a relatively unspecialized cell acquires specialized features of a vestibular hair cell.